spiny bracelet of Nageotte [GO:0097455] (cellular component) References: PMID:15988042 Sources: NIF_Subcellular:sao937871668 Relationships: is a type of glial cell projection [GO:0097386] Definition: Paranodal terminations of Schwann cells that do not directly contact the paranodal axon membrane. Usually found in thicker myelin.